{
  "gene": "UniProtKB:Q9Y6C9",
  "gene_name": "Mitochondrial carrier homolog 2",
  "term_label": "positive regulation of apoptotic process",
  "gene_symbol": "MTCH2",
  "term_id": "GO:0043065"
}